{
  "term_label": "histone binding",
  "gene_name": "Nucleosome assembly protein 1-like 1",
  "gene_symbol": "NAP1L1",
  "gene": "UniProtKB:P55209",
  "term_id": "GO:0042393"
}